alpha-actinin binding [GO:0051393] (molecular function) References: PMID:10984498, PMID:11699871, PMID:15014165 Definition: Binding to alpha-actinin, one of a family of proteins that cross-link F-actin as antiparallel homodimers. Alpha-actinin has a molecular mass of 93-103 KDa; at the N-terminus there are two calponin homology domains, at the C-terminus there are two EF-hands. These two domains are connected by the rod domain. This domain is formed by triple-helical spectrin repeats. Relationships: is a type of actinin binding [GO:0042805] Also known as: alpha-actinin 1 binding, alpha-actinin 4 binding, nonmuscle alpha-actinin binding Subtypes: muscle alpha-actinin binding [GO:0051371]